positive regulation of secretion by cell [GO:1903532] (biological process) Relationships: is a type of positive regulation of cellular process [GO:0048522]; is_a positive regulation of secretion [GO:0051047]; is a type of GO:1903530; positively regulates secretion by cell [GO:0032940] Also known as: positive regulation of cellular secretion, up regulation of cellular secretion, up regulation of secretion by cell, up-regulation of cellular secretion, up-regulation of secretion by cell, upregulation of cellular secretion, upregulation of secretion by cell, activation of cellular secretion, activation of secretion by cell References: PMID:12130530 Sources: GOC:TermGenie, GOC:pm, GO_REF:0000058 Subtypes: positive regulation of neurotransmitter secretion [GO:0001956], positive regulation of extracellular matrix constituent secretion [GO:0003331], positive regulation of glutamate secretion [GO:0014049], positive regulation of serotonin secretion [GO:0014064], positive regulation of prostaglandin secretion [GO:0032308], positive regulation of catecholamine secretion [GO:0033605], positive regulation of exocytosis [GO:0045921], positive regulation of hormone secretion [GO:0046887], positive regulation of protein secretion [GO:0050714], positive regulation of aspartate secretion [GO:1904450] Definition: Any process that activates or increases the frequency, rate or extent of secretion by cell.